{
  "gene_name": "NADH dehydrogenase [ubiquinone] iron-sulfur protein 4, mitochondrial",
  "term_label": "mitochondrial respiratory chain complex I assembly",
  "term_id": "GO:0032981",
  "gene": "UniProtKB:O43181",
  "gene_symbol": "NDUFS4"
}